dCTP catabolic process [GO:0006253] (biological process) Also known as: dCTP breakdown, dCTP catabolism, dCTP degradation Relationships: is a type of GO:0009213; is_a pyrimidine deoxyribonucleotide catabolic process [GO:0009223]; is a type of GO:0046065 Sources: ISBN:0198506732 Definition: The chemical reactions and pathways resulting in the breakdown of dCTP, deoxycytidine triphosphate.